{
  "term_label": "regulation of transcription by RNA polymerase II",
  "term_id": "GO:0006357",
  "gene_name": "Transcription factor Spi-C",
  "gene_symbol": "SPIC",
  "gene": "UniProtKB:Q8N5J4"
}